reproductive senescence [GO:1990636] (biological process) Definition: A life cycle stage during which the reproductive capacity and fitness of an organism declines. References: PMID:24914937, PMID:25523082, PMID:27353257 Also known as: ovarian senescence Note: Note that phases are is_a disjoint from other biological processes. happens_during relationships can operate between phases and other biological processes e.g. DNA replication happens_during S phase. Relationships: is a type of biological phase [GO:0044848] Subtypes: menopause [GO:0042697]